sigma factor antagonist activity [GO:0016989] (molecular function) Also known as: anti-sigma factor activity Relationships: is a type of GO:0003714 Definition: The function of binding to a sigma factor and stopping, preventing or reducing the rate of its transcriptional activity. Sources: GOC:jl, GOC:txnOH, Wikipedia:Anti-sigma_factors